{
  "gene": "UniProtKB:P49902",
  "gene_symbol": "NT5C2",
  "term_label": "Unknown cellular component",
  "term_id": "UNKNOWN:0003",
  "gene_name": "Cytosolic purine 5'-nucleotidase"
}